mitochondrial lrRNA export from mitochondrion [GO:0019091] (biological process) Definition: The process in which a lrRNA, large subunit ribosomal ribonucleic acid, is transported from the mitochondrial matrix into the cytosol. Sources: GOC:ai Also known as: export of mitochondrial lrRNA, mitochondrial lrRNA export, mitochondrial lrRNA export from mitochondria, mitochondrial lrRNA export out of mitochondrion, mitochondrial lrRNA transport from mitochondrion, mitochondrial lrRNA, mitochondrial export Relationships: is a type of mitochondrial rRNA export from mitochondrion [GO:0019090]